delta(3)-delta(2)-enoyl-CoA isomerase activity [GO:0004165] (molecular function) Sources: RHEA:45900 Relationships: is a type of GO:0016863 Also known as: delta3-cis-delta2-trans-enoyl-CoA isomerase, delta3-delta2 enoyl-CoA isomerase activity, dodecenoyl-CoA (3Z)-(2E)-isomerase activity, dodecenoyl-CoA D-isomerase activity, dodecenoyl-CoA delta-isomerase activity, dodecenoyl-CoA delta3-cis-delta2-trans-isomerase activity, 3,2-trans-enoyl-CoA isomerase activity, acetylene-allene isomerase activity, delta(3),delta(2)-enoyl-CoA isomerase activity, delta(3)-cis-delta(2)-trans-enoyl-CoA isomerase activity, delta3,delta2-enoyl-CoA isomerase activity, dodecenoyl-CoA isomerase activity Definition: Catalysis of the reactions: a (3Z)-enoyl-CoA = a 4-saturated (2E)-enoyl-CoA or a (3E)-enoyl-CoA = a 4-saturated (2E)-enoyl-CoA.